{
  "term_label": "positive regulation of activated T cell proliferation",
  "gene": "UniProtKB:P41273",
  "term_id": "GO:0042104",
  "gene_name": "Tumor necrosis factor ligand superfamily member 9",
  "gene_symbol": "TNFSF9"
}